{
  "term_id": "GO:1903426",
  "gene": "UniProtKB:Q9Y2I7",
  "gene_name": "1-phosphatidylinositol 3-phosphate 5-kinase",
  "gene_symbol": "PIKFYVE",
  "term_label": "regulation of reactive oxygen species biosynthetic process"
}